cysteine metabolic process [GO:0006534] (biological process) Definition: The chemical reactions and pathways involving cysteine, 2-amino-3-mercaptopropanoic acid. Subtypes: cysteine catabolic process [GO:0009093], L-asparagine biosynthetic process from cysteine [GO:0019267], cysteine biosynthetic process [GO:0019344], transsulfuration [GO:0019346], GO:0046439 Regulation: regulated by regulation of cysteine metabolic process [GO:1901494] Relationships: is a type of sulfur amino acid metabolic process [GO:0000096]; is a type of alpha-amino acid metabolic process [GO:1901605] Also known as: cysteine metabolism Sources: GOC:go_curators